{
  "term_label": "promoter-specific chromatin binding",
  "term_id": "GO:1990841",
  "gene_name": "Heterogeneous nuclear ribonucleoprotein U",
  "gene_symbol": "HNRNPU",
  "gene": "UniProtKB:Q00839"
}